PKR/eIFalpha signaling [GO:0039585] (biological process) Also known as: EIF2AK2 signal transduction, EIF2AK2/PRK signaling, PKR signal transduction, PKR signaling pathway, signaling through PKR References: PMID:21204021, PMID:22102852, PMID:27629041, PMID:9843495 Sources: VZ:1576 Relationships: is a type of integrated stress response signaling [GO:0140467] Definition: An intracellular signaling cassette that starts with activation and autophosphorylation of PKR (also known as EIF2AK2), which phosphorylates proteins including the translation initiation factor eIF2 to inhibit translation. PKR is activated by stress signals and during the antiviral response, activated by binding to viral double-stranded RNA (dsRNA) leading to inhibition of protein synthesis during viral infection.